regulation of muscle organ development [GO:0048634] (BP) Sources: GOC:go_curators Definition: Any process that modulates the frequency, rate or extent of muscle development. Relationships: is a type of GO:0050793; regulates muscle organ development [GO:0007517] Subtypes: GO:0014708, regulation of striated muscle tissue development [GO:0016202], negative regulation of muscle organ development [GO:0048635], GO:0048636, GO:2000061